regulation of mucus secretion [GO:0070255] (biological process) Definition: Any process that modulates the frequency, rate or extent of the regulated release of mucus from a cell or a tissue. Sources: GOC:add Also known as: regulation of mucus production Relationships: is a type of regulation of body fluid levels [GO:0050878]; is a type of regulation of secretion [GO:0051046]; is a type of GO:0051239; regulates GO:0070254 Subtypes: negative regulation of mucus secretion [GO:0070256], positive regulation of mucus secretion [GO:0070257]